axonemal nexin link [GO:0005931] (cellular component) Also known as: nexin complex, axonemal interdoublet link Relationships: is a type of protein-containing complex [GO:0032991]; BFO_0000050 axoneme [GO:0005930] Definition: A protein complex found in the axoneme of eukaryotic cilia and flagella. It forms interconnections between the microtubule outer doublets that surround the inner central pair of microtubules. References: PMID:21586547, PMID:21728999, PMID:22683354, PMID:9295136 Sources: GOC:cilia, GOC:krc, ISBN:0198506732